{
  "gene": "UniProtKB:Q9H6S3",
  "gene_symbol": "EPS8L2",
  "term_id": "GO:0032587",
  "term_label": "ruffle membrane",
  "gene_name": "Epidermal growth factor receptor kinase substrate 8-like protein 2"
}